heart rudiment morphogenesis [GO:0003314] (biological process) Sources: GOC:mtg_heart Relationships: is_a morphogenesis of an epithelium [GO:0002009]; is a type of embryonic morphogenesis [GO:0048598]; is part of heart morphogenesis [GO:0003007]; is part of GO:0003313 Also known as: heart cone morphogenesis Definition: The process in which the anatomical structures of the heart rudiment are generated and organized.